suture of dorsal opening [GO:0007396] (biological process) Relationships: is a type of embryonic morphogenesis [GO:0048598]; BFO_0000050 dorsal closure [GO:0007391] Definition: Closure of the dorsal hole. Filopodia extending from each leading edge interdigitate at the dorsal midline and appear to prime the formation of adherens junctions between the two rows of leading edge cells. Newly formed septate junctions are also used to seal the dorsal hole. References: PMID:12147138 Sources: GOC:bf